{
  "gene_symbol": "MARCHF7",
  "term_id": "GO:0043130",
  "gene_name": "E3 ubiquitin-protein ligase MARCHF7",
  "gene": "UniProtKB:Q9H992",
  "term_label": "ubiquitin binding"
}